{
  "gene": "UniProtKB:Q5JUK3",
  "term_label": "intracellular sodium-activated potassium channel activity",
  "term_id": "GO:0005228",
  "gene_symbol": "KCNT1",
  "gene_name": "Potassium channel subfamily T member 1"
}